{
  "gene_symbol": "CCNF",
  "gene": "UniProtKB:P41002",
  "term_label": "G1/S transition of mitotic cell cycle",
  "gene_name": "Cyclin-F",
  "term_id": "GO:0000082"
}